{
  "gene": "UniProtKB:Q13454",
  "gene_symbol": "TUSC3",
  "term_id": "UNKNOWN:0001",
  "term_label": "Unknown molecular function",
  "gene_name": "Tumor suppressor candidate 3"
}